metanephric prebend segment development [GO:0072228] (biological process) Sources: GOC:mtg_kidney_jan10 Relationships: is a type of prebend segment development [GO:0072066]; is part of GO:0072220 Definition: The process whose specific outcome is the progression of the metanephric prebend segment over time, from its formation to the mature structure. The metanephric prebend segment is a part of the metanephric descending thin limb that lies before the bend and exhibits permeabilities characteristic of the ascending limb, especially negligible water permeability.